{
  "gene": "UniProtKB:O75578",
  "gene_symbol": "ITGA10",
  "term_id": "GO:0009986",
  "gene_name": "Integrin alpha-10",
  "term_label": "cell surface"
}